response to xenobiotic stimulus [GO:0009410] (biological process) Sources: GOC:jl, GOC:krc Subtypes: cellular response to xenobiotic stimulus [GO:0071466] Definition: Any process that results in a change in state or activity of a cell or an organism (in terms of movement, secretion, enzyme production, gene expression, etc.) as a result of a stimulus from a xenobiotic, a compound foreign to the organism exposed to it. It may be synthesized by another organism (like ampicilin) or it can be a synthetic chemical. Also known as: drug resistance, drug susceptibility/resistance, response to drug Relationships: is a type of response to chemical [GO:0042221] Regulation: regulated by regulation of response to drug [GO:2001023]; negatively regulated by GO:2001024; positively regulated by positive regulation of response to drug [GO:2001025]